{
  "gene_symbol": "COMMD4",
  "gene": "UniProtKB:Q9H0A8",
  "term_id": "UNKNOWN:0003",
  "gene_name": "COMM domain-containing protein 4",
  "term_label": "Unknown cellular component"
}